{
  "gene_symbol": "PCSK2",
  "gene": "UniProtKB:P16519",
  "term_id": "GO:0043005",
  "gene_name": "Neuroendocrine convertase 2",
  "term_label": "neuron projection"
}